{
  "gene": "UniProtKB:O94915",
  "gene_symbol": "FRYL",
  "term_id": "GO:0030427",
  "term_label": "site of polarized growth",
  "gene_name": "Protein furry homolog-like"
}